{
  "term_label": "enzyme inhibitor activity",
  "gene": "UniProtKB:Q9H3M7",
  "term_id": "GO:0004857",
  "gene_name": "Thioredoxin-interacting protein",
  "gene_symbol": "TXNIP"
}